{
  "term_label": "voltage-gated potassium channel complex",
  "gene_symbol": "LRRC52",
  "gene_name": "Leucine-rich repeat-containing protein 52",
  "term_id": "GO:0008076",
  "gene": "UniProtKB:Q8N7C0"
}